myosin VI light chain binding [GO:0070856] (molecular function) Sources: GOC:sart Relationships: is_a myosin light chain binding [GO:0032027]; is a type of GO:0070853 Definition: Binding to a light chain of a myosin VI complex.